{
  "term_id": "UNKNOWN:0002",
  "gene": "UniProtKB:Q8NCU4",
  "gene_symbol": "CCDC191",
  "gene_name": "Coiled-coil domain-containing protein 191",
  "term_label": "Unknown biological process"
}